regulation of Wnt signaling pathway [GO:0030111] (biological process) Definition: Any process that modulates the frequency, rate or extent of the activity of the Wnt signal transduction pathway. Subtypes: regulation of Wnt signaling pathway involved in heart development [GO:0003307], positive regulation of Wnt signaling pathway [GO:0030177], negative regulation of Wnt signaling pathway [GO:0030178], regulation of canonical Wnt signaling pathway [GO:0060828], regulation of non-canonical Wnt signaling pathway [GO:2000050] Also known as: regulation of Wnt receptor signaling pathway, regulation of Wnt receptor signalling pathway, regulation of Wnt-activated signaling pathway, regulation of frizzled signaling pathway, regulation of frizzled signalling pathway Sources: GOC:dph, GOC:mah, GOC:tb Relationships: is a type of regulation of signal transduction [GO:0009966]; regulates Wnt signaling pathway [GO:0016055]